{
  "term_id": "UNKNOWN:0001",
  "term_label": "Unknown molecular function",
  "gene_name": "C-X-C motif chemokine 11",
  "gene": "UniProtKB:O14625",
  "gene_symbol": "CXCL11"
}